{
  "term_label": "melanin biosynthetic process",
  "term_id": "GO:0042438",
  "gene": "UniProtKB:P14679",
  "gene_symbol": "TYR",
  "gene_name": "Tyrosinase"
}